{
  "gene": "UniProtKB:Q6ZTB9",
  "gene_name": "Putative zinc finger protein 833",
  "term_id": "GO:0005634",
  "gene_symbol": "ZNF833P",
  "term_label": "nucleus"
}